regulation of nephron tubule epithelial cell differentiation [GO:0072182] (biological process) Sources: GOC:mtg_kidney_jan10 Subtypes: negative regulation of nephron tubule epithelial cell differentiation [GO:0072183], regulation of metanephric nephron tubule epithelial cell differentiation [GO:0072307], regulation of mesonephric nephron tubule epithelial cell differentiation [GO:2000093], positive regulation of nephron tubule epithelial cell differentiation [GO:2000768] Definition: Any process that modulates the frequency, rate or extent of nephron tubule epithelial cell differentiation. Relationships: is a type of GO:2000696; regulates nephron tubule epithelial cell differentiation [GO:0072160]